negative regulation of hematopoietic progenitor cell differentiation [GO:1901533] (biological process) Also known as: down regulation of haematopoietic progenitor cell differentiation, down regulation of haemopoietic progenitor cell differentiation, down regulation of hemopoietic progenitor cell differentiation, down-regulation of haematopoietic progenitor cell differentiation, down-regulation of haemopoietic progenitor cell differentiation, down-regulation of hemopoietic progenitor cell differentiation, downregulation of haematopoietic progenitor cell differentiation, downregulation of haemopoietic progenitor cell differentiation, downregulation of hemopoietic progenitor cell differentiation, inhibition of haematopoietic progenitor cell differentiation, inhibition of haemopoietic progenitor cell differentiation, negative regulation of haematopoietic progenitor cell differentiation, negative regulation of haemopoietic progenitor cell differentiation, negative regulation of hemopoietic progenitor cell differentiation, inhibition of hemopoietic progenitor cell differentiation, down regulation of hematopoietic progenitor cell differentiation, down-regulation of hematopoietic progenitor cell differentiation, downregulation of hematopoietic progenitor cell differentiation, inhibition of hematopoietic progenitor cell differentiation Relationships: is a type of negative regulation of cell differentiation [GO:0045596]; is a type of regulation of hematopoietic progenitor cell differentiation [GO:1901532]; negatively regulates hematopoietic progenitor cell differentiation [GO:0002244] Subtypes: negative regulation of hematopoietic stem cell differentiation [GO:1902037], negative regulation of myeloid progenitor cell differentiation [GO:1905454], negative regulation of lymphoid progenitor cell differentiation [GO:1905457] Definition: Any process that stops, prevents or reduces the frequency, rate or extent of hematopoietic progenitor cell differentiation. Sources: GOC:BHF, GOC:TermGenie, GOC:rl